{
  "term_id": "GO:0006396",
  "term_label": "RNA processing",
  "gene_symbol": "ADAR",
  "gene": "UniProtKB:P55265",
  "gene_name": "Double-stranded RNA-specific adenosine deaminase"
}